broad specificity neutral L-amino acid:basic L-amino acid antiporter activity [GO:0180009] (molecular function) Definition: Enables the transfer of a solute or solutes from one side of a membrane to the other according to the reaction: basic L-amino acid(in) + neutral L-amino acid(out) = basic L-amino acid(in) + neutral L-amino acid(out). References: PMID:23506863, PMID:8663357 Also known as: neutral L-amino acid:cationic L-amino acid antiporter activity, neutral L-amino acid:dibasic L-amino acid antiporter activity, neutral L-amino acid:positively-charged polar L-amino acid antiporter activity, system b(0,+)-type activity Relationships: is a type of basic amino acid transmembrane transporter activity [GO:0015174]; is a type of neutral L-amino acid transmembrane transporter activity [GO:0015175]; is a type of antiporter activity [GO:0015297]